glutamine-phenylpyruvate transaminase activity [GO:0047316] (molecular function) Relationships: is a type of L-glutamine aminotransferase activity [GO:0070548] Definition: Catalysis of the reaction: keto-phenylpyruvate + L-glutamine = 2-oxoglutaramate + L-phenylalanine. Also known as: glutamine-phenylpyruvate aminotransferase activity, L-glutamine:phenylpyruvate aminotransferase activity, glutamine transaminase K activity, glutamine--phenylpyruvate aminotransferase activity Sources: EC:2.6.1.64, RHEA:17593